{
  "gene_symbol": "LINC01545",
  "term_id": "UNKNOWN:0003",
  "gene_name": "Putative uncharacterized protein encoded by LINC01545",
  "term_label": "Unknown cellular component",
  "gene": "UniProtKB:Q5VT33"
}